{
  "gene": "UniProtKB:Q5RIA9",
  "gene_symbol": "ZNG1E",
  "gene_name": "Zinc-regulated GTPase metalloprotein activator 1E",
  "term_label": "cytoplasm",
  "term_id": "GO:0005737"
}